{
  "gene_name": "Nonsense-mediated mRNA decay factor SMG9",
  "term_id": "UNKNOWN:0001",
  "term_label": "Unknown molecular function",
  "gene_symbol": "SMG9",
  "gene": "UniProtKB:Q9H0W8"
}